{
  "term_label": "cilium assembly",
  "gene_symbol": "IFT80",
  "gene": "UniProtKB:Q9P2H3",
  "term_id": "GO:0060271",
  "gene_name": "Intraflagellar transport protein 80 homolog"
}